alpha-beta T cell activation involved in immune response [GO:0002287] (biological process) Relationships: is a type of GO:0002286; is a type of alpha-beta T cell activation [GO:0046631] Sources: GOC:add, ISBN:0781735149 Also known as: alpha-beta T cell activation during immune response, alpha-beta T lymphocyte activation during immune response, alpha-beta T-cell activation during immune response, alpha-beta T-lymphocyte activation during immune response Definition: The change in morphology and behavior of an alpha-beta T cell resulting from exposure to a mitogen, cytokine, chemokine, cellular ligand, or an antigen for which it is specific, leading to the initiation or perpetuation of an immune response. Subtypes: GO:0002288, GO:0002293, alpha-beta T cell proliferation involved in immune response [GO:0002310]